{
  "gene": "UniProtKB:O95295",
  "gene_symbol": "SNAPIN",
  "gene_name": "SNARE-associated protein Snapin",
  "term_id": "GO:0032418",
  "term_label": "lysosome localization"
}